{
  "gene": "UniProtKB:Q86YM7",
  "term_id": "GO:2001256",
  "gene_name": "Homer protein homolog 1",
  "term_label": "regulation of store-operated calcium entry",
  "gene_symbol": "HOMER1"
}